{
  "gene_name": "Translation machinery-associated protein 7",
  "gene_symbol": "TMA7",
  "term_id": "UNKNOWN:0003",
  "gene": "UniProtKB:Q9Y2S6",
  "term_label": "Unknown cellular component"
}